{
  "gene_symbol": "EME1",
  "gene_name": "Crossover junction endonuclease EME1",
  "term_id": "GO:0031297",
  "gene": "UniProtKB:Q96AY2",
  "term_label": "replication fork processing"
}